{
  "gene_name": "Aprataxin and PNK-like factor",
  "term_label": "site of double-strand break",
  "term_id": "GO:0035861",
  "gene": "UniProtKB:Q8IW19",
  "gene_symbol": "APLF"
}